{
  "gene": "UniProtKB:Q6PUV4",
  "term_id": "GO:0043195",
  "gene_symbol": "CPLX2",
  "gene_name": "Complexin-2",
  "term_label": "terminal bouton"
}